regulation of p38MAPK cascade [GO:1900744] (biological process) Also known as: regulation of p38 MAPK cascade, regulation of p38 cascade, regulation of osmosensory signaling MAPK cascade Sources: GOC:TermGenie Definition: Any process that modulates the frequency, rate or extent of p38MAPK cascade. Relationships: is a type of regulation of MAPK cascade [GO:0043408]; RO_0002211 p38MAPK cascade [GO:0038066] Subtypes: GO:1900745, negative regulation of p38MAPK cascade [GO:1903753]